ATPase-coupled nonpolar-amino acid transporter activity [GO:0015425] (molecular function) Definition: Enables the transfer of a solute or solutes from one side of a membrane to the other according to the reaction: ATP + H2O + nonpolar amino acid(out) = ADP + phosphate + nonpolar amino acid(in). Sources: EC:7.4.2.2 Also known as: ATP-dependent nonpolar-amino acid transporter activity, nonpolar amino acid-transporting ATPase activity, nonpolar-amino acid ABC transporter, nonpolar-amino acid-transporting ATPase activity, nonpolar-amino-acid-transporting ATPase activity, leucine/isoleucine/valine porter activity Relationships: is a type of ABC-type amino acid transporter activity [GO:0015424]